{
  "term_id": "GO:0019731",
  "term_label": "antibacterial humoral response",
  "gene_symbol": "H2BC3",
  "gene_name": "Histone H2B type 1-B",
  "gene": "UniProtKB:P33778"
}